{
  "gene_symbol": "CASP8",
  "term_label": "CD95 death-inducing signaling complex",
  "gene_name": "Caspase-8",
  "term_id": "GO:0031265",
  "gene": "UniProtKB:Q14790"
}